xylitol kinase activity [GO:0050400] (molecular function) Sources: EC:2.7.1.122, RHEA:20209 Also known as: ATP:xylitol 5-phosphotransferase activity, xylitol phosphotransferase activity Relationships: is a type of kinase activity [GO:0016301]; is_a phosphotransferase activity, alcohol group as acceptor [GO:0016773] Definition: Catalysis of the reaction: ATP + xylitol = ADP + 2 H+ + xylitol 5-phosphate.